pollen intine formation [GO:0160030] (biological process) Definition: Formation of pollen intine, the inner layer of the pollen wall. The reticulate pollen wall pattern consists of two layers, exine and intine. References: PMID:35498668 Relationships: is a type of pollen wall assembly [GO:0010208]